male genitalia development [GO:0030539] (biological process) Definition: The process whose specific outcome is the progression of the male genitalia over time, from its formation to the mature structure. Also known as: male genital development Relationships: is a type of genitalia development [GO:0048806]; is a type of reproductive system development [GO:0061458]; is part of male sex differentiation [GO:0046661] Sources: GOC:ems, ISBN:0140512888